thyroid hormone transmembrane transporter activity [GO:0015349] (molecular function) Relationships: is a type of secondary active transmembrane transporter activity [GO:0015291]; is part of GO:0070327 Sources: GOC:ai Definition: Enables the transfer of thyroid hormones from one side of a membrane to the other. Thyroid hormone are any of the compounds secreted by the thyroid gland, largely thyroxine and triiodothyronine.